{
  "gene": "UniProtKB:P98170",
  "term_id": "GO:0005634",
  "term_label": "nucleus",
  "gene_symbol": "XIAP",
  "gene_name": "E3 ubiquitin-protein ligase XIAP"
}